{
  "gene": "UniProtKB:P29322",
  "gene_symbol": "EPHA8",
  "term_label": "transmembrane-ephrin receptor activity",
  "gene_name": "Ephrin type-A receptor 8",
  "term_id": "GO:0005005"
}